{
  "gene": "UniProtKB:B9A6J9",
  "gene_symbol": "TBC1D3L",
  "term_label": "GTPase activator activity",
  "term_id": "GO:0005096",
  "gene_name": "TBC1 domain family member 3L"
}